regulation of CD8-positive, alpha-beta T cell extravasation [GO:2000449] (biological process) Definition: Any process that modulates the frequency, rate or extent of CD8-positive, alpha-beta T cell extravasation. Subtypes: negative regulation of CD8-positive, alpha-beta T cell extravasation [GO:2000450], positive regulation of CD8-positive, alpha-beta T cell extravasation [GO:2000451], regulation of CD8-positive, alpha-beta cytotoxic T cell extravasation [GO:2000452], regulation of T-helper 17 cell extravasation [GO:2000455] Sources: GOC:obol Relationships: is a type of GO:2000407; regulates CD8-positive, alpha-beta T cell extravasation [GO:0035697]